F2-isoprostane catabolic process [GO:0062233] (biological process) Relationships: is a type of GO:1901523 References: PMID:16371369, PMID:25449649 Definition: The chemical reactions and pathways resulting in the breakdown of F2-isoprostane.